{
  "gene_symbol": "TAS2R40",
  "term_label": "detection of chemical stimulus involved in sensory perception of bitter taste",
  "term_id": "GO:0001580",
  "gene_name": "Taste receptor type 2 member 40",
  "gene": "UniProtKB:P59535"
}